{
  "term_id": "GO:0005549",
  "gene_name": "Olfactory receptor 5M9",
  "gene": "UniProtKB:Q8NGP3",
  "gene_symbol": "OR5M9",
  "term_label": "odorant binding"
}